stem cell fate determination [GO:0048867] (biological process) Sources: CL:0000034, GOC:isa_complete Definition: The process in which a cell becomes capable of differentiating autonomously into a stem cell regardless of its environment; upon determination, the cell fate cannot be reversed. Subtypes: neural crest cell fate determination [GO:0014035], skeletal muscle satellite cell fate determination [GO:0014818] Relationships: is a type of cell fate determination [GO:0001709]; is part of stem cell fate commitment [GO:0048865]